{
  "term_id": "GO:0070888",
  "gene_name": "Neurogenic differentiation factor 1",
  "term_label": "E-box binding",
  "gene_symbol": "NEUROD1",
  "gene": "UniProtKB:Q13562"
}